negative regulation of gastrulation [GO:2000542] (biological process) Relationships: is a type of GO:0010470; is a type of negative regulation of embryonic development [GO:0045992]; RO_0002212 gastrulation [GO:0007369] Definition: Any process that stops, prevents or reduces the frequency, rate or extent of gastrulation. Sources: GOC:obol